adenosylselenohomocysteinase activity [GO:0098604] (MF) Relationships: is a type of trialkylsulfonium hydrolase activity [GO:0016802] Definition: Catalysis of the reaction: Se-Adenosyl-L-selenohomocysteine + H2O = Adenosine + Selenohomocysteine. References: PMID:1711890, PMID:7305945 Sources: GOC:dos